{
  "gene_symbol": "TLR7",
  "term_label": "toll-like receptor signaling pathway",
  "gene_name": "Toll-like receptor 7",
  "term_id": "GO:0002224",
  "gene": "UniProtKB:Q9NYK1"
}